{
  "gene": "UniProtKB:Q9BZJ7",
  "gene_name": "G-protein coupled receptor 62",
  "term_label": "receptor complex",
  "term_id": "GO:0043235",
  "gene_symbol": "GPR62"
}